box C/D sno(s)RNA binding [GO:0034512] (molecular function) Sources: GOC:mah Also known as: box C/D sRNA binding, box C/D snoRNA binding Relationships: is a type of snoRNA binding [GO:0030515] Definition: Binding to a box C/D small nucleolar RNA.